negative regulation of post-translational protein modification [GO:1901874] (biological process) Definition: Any process that stops, prevents or reduces the frequency, rate or extent of post-translational protein modification. References: PMID:21209915 Sources: GOC:TermGenie, GOC:yaf Also known as: down regulation of PTM, down regulation of post-translational amino acid modification, down regulation of post-translational modification, down regulation of post-translational protein modification, down regulation of posttranslational amino acid modification, down regulation of posttranslational modification, down regulation of posttranslational protein modification, down-regulation of PTM, down-regulation of post-translational amino acid modification, down-regulation of post-translational modification, down-regulation of post-translational protein modification, down-regulation of posttranslational amino acid modification, down-regulation of posttranslational modification, down-regulation of posttranslational protein modification, downregulation of PTM, downregulation of post-translational amino acid modification, downregulation of post-translational modification, downregulation of post-translational protein modification, downregulation of posttranslational amino acid modification, downregulation of posttranslational modification, downregulation of posttranslational protein modification, inhibition of PTM, inhibition of post-translational amino acid modification, inhibition of post-translational modification, inhibition of posttranslational amino acid modification, inhibition of posttranslational modification, inhibition of posttranslational protein modification, negative regulation of PTM, negative regulation of post-translational amino acid modification, negative regulation of post-translational modification, negative regulation of posttranslational amino acid modification, negative regulation of posttranslational modification, negative regulation of posttranslational protein modification, inhibition of post-translational protein modification Relationships: is a type of GO:0031400; is a type of regulation of post-translational protein modification [GO:1901873]; negatively regulates post-translational protein modification [GO:0043687] Subtypes: negative regulation of protein modification by small protein conjugation or removal [GO:1903321]